{
  "term_id": "GO:0004830",
  "gene_symbol": "WARS1",
  "term_label": "tryptophan-tRNA ligase activity",
  "gene": "UniProtKB:P23381",
  "gene_name": "Tryptophan--tRNA ligase, cytoplasmic"
}